{
  "gene_symbol": "LMNB2",
  "gene": "UniProtKB:Q03252",
  "gene_name": "Lamin-B2",
  "term_id": "GO:0006998",
  "term_label": "nuclear envelope organization"
}